{
  "term_label": "Unknown cellular component",
  "term_id": "UNKNOWN:0003",
  "gene_symbol": "TTC34",
  "gene_name": "Tetratricopeptide repeat protein 34",
  "gene": "UniProtKB:A8MYJ7"
}